G/U mismatch-specific uracil-DNA glycosylase activity [GO:0043739] (molecular function) Relationships: is a type of uracil DNA N-glycosylase activity [GO:0004844]; is a type of pyrimidine-specific mismatch base pair DNA N-glycosylase activity [GO:0008263] Also known as: uracil mismatch repair protein, GU mismatch-specific uracil-DNA glycosylase activity, MUG Definition: Hydrolyzes mismatched double-stranded DNA and polynucleotides, releasing free uracil and leaving an apyrimidinic (AP) site. References: PMID:24739389 Sources: EC:3.2.2.28